positive regulation of mature B cell apoptotic process [GO:0002907] (BP) Definition: Any process that activates or increases the frequency, rate, or extent of mature B cell apoptotic process. Sources: GOC:add, GOC:mtg_apoptosis Also known as: up regulation of mature B cell apoptosis, up-regulation of mature B cell apoptosis, upregulation of mature B cell apoptosis, activation of mature B cell apoptosis, positive regulation of mature B cell apoptosis, stimulation of mature B cell apoptosis Relationships: is a type of positive regulation of immune system process [GO:0002684]; is a type of positive regulation of B cell apoptotic process [GO:0002904]; is a type of regulation of mature B cell apoptotic process [GO:0002905]; positively regulates mature B cell apoptotic process [GO:0002901]